{
  "gene_symbol": "MEF2D",
  "term_id": "GO:0000981",
  "gene": "UniProtKB:Q14814",
  "term_label": "DNA-binding transcription factor activity, RNA polymerase II-specific",
  "gene_name": "Myocyte-specific enhancer factor 2D"
}